{
  "gene": "UniProtKB:O95900",
  "gene_symbol": "TRUB2",
  "term_label": "pseudouridine synthase activity",
  "gene_name": "Pseudouridylate synthase TRUB2, mitochondrial",
  "term_id": "GO:0009982"
}